positive regulation of inner ear receptor cell differentiation [GO:2000982] (biological process) Subtypes: positive regulation of inner ear auditory receptor cell differentiation [GO:0045609] Relationships: is a type of positive regulation of mechanoreceptor differentiation [GO:0045633]; is a type of regulation of inner ear receptor cell differentiation [GO:2000980]; positively regulates inner ear receptor cell differentiation [GO:0060113] Definition: Any process that activates or increases the frequency, rate or extent of inner ear receptor cell differentiation. Also known as: positive regulation of inner ear hair cell differentiation Sources: GOC:obol